{
  "term_label": "Golgi-associated vesicle membrane",
  "term_id": "GO:0030660",
  "gene_symbol": "SPPL2B",
  "gene": "UniProtKB:Q8TCT7",
  "gene_name": "Signal peptide peptidase-like 2B"
}